{
  "term_label": "cytokine activity",
  "gene": "UniProtKB:P61812",
  "term_id": "GO:0005125",
  "gene_symbol": "TGFB2",
  "gene_name": "Transforming growth factor beta-2 proprotein"
}